{
  "term_label": "Unknown molecular function",
  "gene_name": "Protein FAM182A",
  "gene": "UniProtKB:Q5T1J6",
  "gene_symbol": "FAM182A",
  "term_id": "UNKNOWN:0001"
}